{
  "gene_name": "Ras-specific guanine nucleotide-releasing factor RalGPS2",
  "gene_symbol": "RALGPS2",
  "term_id": "GO:0005886",
  "term_label": "plasma membrane",
  "gene": "UniProtKB:Q86X27"
}